ganglioside metabolic process [GO:0001573] (biological process) Also known as: ganglioside metabolism Sources: ISBN:0198506732 Definition: The chemical reactions and pathways involving ceramide oligosaccharides carrying in addition to other sugar residues, one or more sialic acid residues. Relationships: is a type of ceramide metabolic process [GO:0006672]; is_a GO:0006687 Subtypes: ganglioside biosynthetic process [GO:0001574], GO:0006689